{
  "term_label": "Unknown cellular component",
  "term_id": "UNKNOWN:0003",
  "gene_name": "Basal body-orientation factor 1",
  "gene_symbol": "BBOF1",
  "gene": "UniProtKB:Q8ND07"
}